{
  "gene_name": "Peptidyl-prolyl cis-trans isomerase G",
  "gene": "UniProtKB:Q13427",
  "term_label": "cytoplasm",
  "gene_symbol": "PPIG",
  "term_id": "GO:0005737"
}